{
  "term_id": "GO:0051562",
  "term_label": "negative regulation of mitochondrial calcium ion concentration",
  "gene_name": "Fetal and adult testis-expressed transcript protein",
  "gene_symbol": "FATE1",
  "gene": "UniProtKB:Q969F0"
}